{
  "gene_name": "Unconventional myosin-Ic",
  "gene": "UniProtKB:O00159",
  "gene_symbol": "MYO1C",
  "term_label": "microvillus",
  "term_id": "GO:0005902"
}